{
  "gene_name": "HLA class I histocompatibility antigen, alpha chain F",
  "gene": "UniProtKB:P30511",
  "term_id": "GO:0002486",
  "gene_symbol": "HLA-F",
  "term_label": "antigen processing and presentation of endogenous peptide antigen via MHC class I via ER pathway, TAP-independent"
}